{
  "gene_name": "Coatomer subunit delta",
  "term_label": "Unknown molecular function",
  "gene": "UniProtKB:P48444",
  "gene_symbol": "ARCN1",
  "term_id": "UNKNOWN:0001"
}